{
  "gene_symbol": "MRM1",
  "term_label": "rRNA modification",
  "term_id": "GO:0000154",
  "gene_name": "rRNA methyltransferase 1, mitochondrial",
  "gene": "UniProtKB:Q6IN84"
}